{
  "gene": "UniProtKB:Q9BQ52",
  "term_id": "GO:0005739",
  "term_label": "mitochondrion",
  "gene_symbol": "ELAC2",
  "gene_name": "Zinc phosphodiesterase ELAC protein 2"
}